{
  "gene": "UniProtKB:Q92622",
  "term_label": "late endosome",
  "term_id": "GO:0005770",
  "gene_name": "Run domain Beclin-1-interacting and cysteine-rich domain-containing protein",
  "gene_symbol": "RUBCN"
}